dendrite development [GO:0016358] (biological process) Definition: The process whose specific outcome is the progression of the dendrite over time, from its formation to the mature structure. Regulation: regulated by regulation of dendrite development [GO:0050773]; positively regulated by positive regulation of dendrite development [GO:1900006]; negatively regulated by negative regulation of dendrite development [GO:2000171] Subtypes: dendrite development by retrograde extension [GO:0003390], dendrite regeneration [GO:0031104], basal dendrite development [GO:0150018], GO:0150022 References: PMID:22683681 Sources: GOC:aruk, GOC:bc, GOC:jl, ISBN:0198506732 Relationships: is a type of neuron projection development [GO:0031175]; is a type of anatomical structure development [GO:0048856]